{
  "term_id": "GO:0032872",
  "gene_name": "Tumor necrosis factor receptor superfamily member 6",
  "gene": "UniProtKB:P25445",
  "gene_symbol": "FAS",
  "term_label": "regulation of stress-activated MAPK cascade"
}